{
  "gene": "UniProtKB:Q9H2F3",
  "term_id": "UNKNOWN:0002",
  "term_label": "Unknown biological process",
  "gene_symbol": "HSD3B7",
  "gene_name": "3 beta-hydroxysteroid dehydrogenase type 7"
}